{
  "term_id": "UNKNOWN:0001",
  "gene_name": "Lysosome-associated membrane glycoprotein 2",
  "term_label": "Unknown molecular function",
  "gene": "UniProtKB:P13473",
  "gene_symbol": "LAMP2"
}